physiological muscle hypertrophy [GO:0003298] (biological process) Definition: The enlargement or overgrowth of all or part of a muscle organ or tissue due to an increase in the size of its muscle cells. Physiological hypertrophy is a normal process during development. Sources: GOC:mtg_heart Relationships: is a type of muscle hypertrophy [GO:0014896] Subtypes: physiological cardiac muscle hypertrophy [GO:0003301]